{
  "gene_symbol": "CCDC57",
  "term_id": "GO:0007020",
  "gene": "UniProtKB:Q2TAC2",
  "term_label": "microtubule nucleation",
  "gene_name": "Coiled-coil domain-containing protein 57"
}